H1-4K26 methyltransferase activity [GO:0140189] (molecular function) Relationships: is a type of histone H1 methyltransferase activity [GO:0140188] Definition: Catalysis of the reaction: S-adenosyl-L-methionine + histone H1-4 L-lysine (position 26) = S-adenosyl-L-homocysteine + histone H1-4 N6-methyl-L-lysine (position 26). References: PMID:19144645